{
  "term_id": "UNKNOWN:0001",
  "gene_name": "V-set and immunoglobulin domain-containing protein 1",
  "gene_symbol": "VSIG1",
  "gene": "UniProtKB:Q86XK7",
  "term_label": "Unknown molecular function"
}